{
  "gene": "UniProtKB:Q30154",
  "term_id": "GO:0050778",
  "gene_name": "HLA class II histocompatibility antigen, DR beta 5 chain",
  "term_label": "positive regulation of immune response",
  "gene_symbol": "HLA-DRB5"
}